actomyosin [GO:0042641] (cellular component) Also known as: actomyosin complex, actomyosin structure Definition: Any complex of actin, myosin, and accessory proteins. Sources: GOC:go_curators Relationships: is a type of GO:0110165; is part of actin cytoskeleton [GO:0015629] Subtypes: stress fiber [GO:0001725]